cellular response to resveratrol [GO:1904639] (biological process) Relationships: is a type of cellular response to oxygen-containing compound [GO:1901701]; is a type of response to resveratrol [GO:1904638] Definition: Any process that results in a change in state or activity of a cell (in terms of movement, secretion, enzyme production, gene expression, etc.) as a result of a resveratrol stimulus. References: PMID:23555824 Sources: GOC:TermGenie, GO_REF:0000071